negative regulation of cell adhesion mediated by integrin [GO:0033629] (biological process) Definition: Any process that stops, prevents, or reduces the frequency, rate, or extent of cell adhesion mediated by integrin. Also known as: negative regulation of cell adhesion mediated by integrin complex Sources: GOC:add Relationships: is a type of negative regulation of cell adhesion [GO:0007162]; is_a regulation of cell adhesion mediated by integrin [GO:0033628]; negatively regulates cell adhesion mediated by integrin [GO:0033627] Subtypes: negative regulation of cell-cell adhesion mediated by integrin [GO:0033633]